{
  "gene_name": "Protein phosphatase 1 regulatory subunit 26",
  "gene": "UniProtKB:Q5T8A7",
  "term_label": "Unknown biological process",
  "term_id": "UNKNOWN:0002",
  "gene_symbol": "PPP1R26"
}